{
  "gene_name": "Keratin, type I cytoskeletal 12",
  "term_label": "structural constituent of skin epidermis",
  "gene": "UniProtKB:Q99456",
  "gene_symbol": "KRT12",
  "term_id": "GO:0030280"
}